{
  "gene_name": "Protein stum homolog",
  "gene_symbol": "STUM",
  "term_id": "UNKNOWN:0002",
  "term_label": "Unknown biological process",
  "gene": "UniProtKB:Q69YW2"
}